positive regulation of tRNA C5-cytosine methylation [GO:0110005] (biological process) References: PMID:23074192 Sources: GOC:vw Definition: Any process that activates or increases the frequency, rate or extent of tRNA C5-cytosine methylation. Relationships: is a type of GO:0110003; is_a positive regulation of tRNA methylation [GO:0110004]; positively regulates tRNA C5-cytosine methylation [GO:0002946]